negative regulation of toluene catabolic process [GO:1901435] (biological process) Definition: Any process that stops, prevents or reduces the frequency, rate or extent of toluene catabolic process. Sources: GOC:TermGenie, GOC:mengo_curators Also known as: down regulation of toluene breakdown, down regulation of toluene catabolic process, down regulation of toluene catabolism, down regulation of toluene degradation, down-regulation of toluene breakdown, down-regulation of toluene catabolic process, down-regulation of toluene catabolism, down-regulation of toluene degradation, downregulation of toluene breakdown, downregulation of toluene catabolic process, downregulation of toluene catabolism, downregulation of toluene degradation, inhibition of toluene breakdown, inhibition of toluene catabolism, inhibition of toluene degradation, negative regulation of toluene breakdown, negative regulation of toluene catabolism, negative regulation of toluene degradation, inhibition of toluene catabolic process Relationships: is a type of GO:0009895; is a type of regulation of toluene catabolic process [GO:1901434]; negatively regulates toluene catabolic process [GO:0042203]